{
  "term_id": "UNKNOWN:0001",
  "gene_name": "Protein TFG",
  "term_label": "Unknown molecular function",
  "gene_symbol": "TFG",
  "gene": "UniProtKB:Q92734"
}